nuclear speck [GO:0016607] (cellular component) Definition: A discrete extra-nucleolar subnuclear domain, 20-50 in number, in which splicing factors are seen to be localized by immunofluorescence microscopy. References: PMID:28977640 Also known as: nuclear speckle, nuclear speckles, splicing speckle, speckle domain, speckle focus Relationships: is a type of GO:0140168 Subtypes: GO:0035062